{
  "gene": "UniProtKB:B7ZAQ6",
  "gene_name": "Golgi pH regulator A",
  "term_id": "GO:0032580",
  "gene_symbol": "GPR89A",
  "term_label": "Golgi cisterna membrane"
}